male anatomical structure morphogenesis [GO:0090598] (biological process) Definition: The processes by which anatomical structures that are only present in the male organism are generated and organized. Sources: GOC:kmv, GOC:tb Relationships: is a type of GO:0009653; is part of male sex differentiation [GO:0046661] Subtypes: nematode male tail tip morphogenesis [GO:0045138], male genitalia morphogenesis [GO:0048808]